{
  "gene_name": "Bifunctional polynucleotide phosphatase_kinase",
  "gene_symbol": "PNKP",
  "term_id": "GO:0005634",
  "gene": "UniProtKB:Q96T60",
  "term_label": "nucleus"
}